{
  "gene": "UniProtKB:P58294",
  "term_id": "UNKNOWN:0001",
  "gene_symbol": "PROK1",
  "term_label": "Unknown molecular function",
  "gene_name": "Prokineticin-1"
}